{
  "term_label": "Golgi apparatus",
  "gene_symbol": "STK26",
  "gene": "UniProtKB:Q9P289",
  "gene_name": "Serine_threonine-protein kinase 26",
  "term_id": "GO:0005794"
}